{
  "term_label": "Unknown cellular component",
  "gene_name": "Hyaluronan mediated motility receptor",
  "gene": "UniProtKB:O75330",
  "gene_symbol": "HMMR",
  "term_id": "UNKNOWN:0003"
}